{
  "term_label": "signal transduction",
  "term_id": "GO:0007165",
  "gene_name": "Receptor-type tyrosine-protein phosphatase C",
  "gene_symbol": "PTPRC",
  "gene": "UniProtKB:P08575"
}